{
  "term_id": "GO:0035091",
  "gene_name": "Pleckstrin homology domain-containing family F member 1",
  "gene": "UniProtKB:Q96S99",
  "term_label": "phosphatidylinositol binding",
  "gene_symbol": "PLEKHF1"
}